{
  "term_label": "microtubule-based movement",
  "gene_symbol": "TCTE1",
  "term_id": "GO:0007018",
  "gene": "UniProtKB:Q5JU00",
  "gene_name": "Dynein regulatory complex subunit 5"
}